{
  "term_id": "UNKNOWN:0002",
  "gene_name": "T cell receptor beta joining 2-5",
  "gene_symbol": "TRBJ2-5",
  "gene": "UniProtKB:A0A0A0MTA4",
  "term_label": "Unknown biological process"
}